{
  "term_id": "UNKNOWN:0002",
  "gene_name": "A-kinase anchor protein 2",
  "term_label": "Unknown biological process",
  "gene": "UniProtKB:Q9Y2D5",
  "gene_symbol": "AKAP2"
}